{
  "gene": "UniProtKB:Q96F05",
  "term_id": "UNKNOWN:0002",
  "term_label": "Unknown biological process",
  "gene_name": "Uncharacterized protein C11orf24",
  "gene_symbol": "C11orf24"
}